{
  "gene_symbol": "ARHGAP44",
  "gene": "UniProtKB:Q17R89",
  "gene_name": "Rho GTPase-activating protein 44",
  "term_id": "GO:0014069",
  "term_label": "postsynaptic density"
}